{
  "term_label": "sphingosine N-acyltransferase activity",
  "gene_symbol": "CERS3",
  "term_id": "GO:0050291",
  "gene": "UniProtKB:Q8IU89",
  "gene_name": "Ceramide synthase 3"
}